{
  "gene_name": "Nucleoside diphosphate kinase, mitochondrial",
  "term_id": "UNKNOWN:0002",
  "term_label": "Unknown biological process",
  "gene": "UniProtKB:O00746",
  "gene_symbol": "NME4"
}